Cus cation efflux complex [GO:1990398] (cellular component) Definition: Transmembrane complex that mediates resistance to copper and silver by cation efflux directly from the cell using the proton-motive force. Spans the inner membrane, periplasm, and outer membrane. Primarily activated under anaerobic conditions by CusR and CusS but also expressed under extreme copper stress, in aerobic growth. Note: An example of this is CusA in E. coli (UniProt symbol P38054) in PMID:23122209. Relationships: is a type of GO:0098797; is a type of copper ion transmembrane transporter complex [GO:1903113]; is a type of silver ion transmembrane transporter complex [GO:1903114] Also known as: Cus cation efflux system, copper efflux complex, copper efflux system, silver efflux complex, silver efflux system References: PMID:23122209 Sources: GOC:bhm